{
  "term_id": "GO:0007165",
  "gene_symbol": "LMBR1",
  "gene": "UniProtKB:Q8WVP7",
  "gene_name": "Limb region 1 protein homolog",
  "term_label": "signal transduction"
}